{
  "gene": "UniProtKB:Q6Y288",
  "term_label": "Unknown cellular component",
  "term_id": "UNKNOWN:0003",
  "gene_symbol": "B3GLCT",
  "gene_name": "Beta-1,3-glucosyltransferase"
}